rRNA pseudouridine synthase activity [GO:0120159] (molecular function) Definition: Catalysis of the reaction: a uridine in rRNA = a pseudouridine in rRNA. Conversion of uridine in an rRNA molecule to pseudouridine by rotation of the C1'-N-1 glycosidic bond of uridine in RNA to a C1'-C5. Relationships: is a type of pseudouridine synthase activity [GO:0009982]; is a type of catalytic activity, acting on RNA [GO:0140098] References: PMID:28432181 Sources: RHEA:54568 Subtypes: GO:0160136, 23S rRNA pseudouridine(2457) synthase activity [GO:0160137], 23S rRNA pseudouridine(2604) synthase activity [GO:0160138], GO:0160139, 23S rRNA pseudouridine(1911/1915/1917) synthase activity [GO:0160140], GO:0160141, 23S rRNA pseudouridine(746) synthase activity [GO:0160142], GO:0160143